{
  "term_label": "double-strand break repair via homologous recombination",
  "term_id": "GO:0000724",
  "gene_name": "DNA repair protein RAD51 homolog 4",
  "gene_symbol": "RAD51D",
  "gene": "UniProtKB:O75771"
}